regulatory T cell differentiation [GO:0045066] (BP) Regulation: regulated by GO:0045589; negatively regulated by negative regulation of regulatory T cell differentiation [GO:0045590]; positively regulated by positive regulation of regulatory T cell differentiation [GO:0045591] Note: Note that immunologists typically use the word 'development' to refer to cells of B or T cell lineages undergoing the process that GO describes as 'cell differentiation'. Definition: The process in which a relatively unspecialized T cell acquires specialized features of a regulatory T cell. Regulatory T cells control or suppress immune responses through a variety of mechanisms and subsets include the CD4+CD25+ cell type as well as certain CD8+ cell types. Also known as: regulatory T lymphocyte differentiation, regulatory T-cell differentiation, regulatory T-lymphocyte differentiation, suppressor T cell differentiation, suppressor T lymphocyte differentiation, suppressor T-cell differentiation, suppressor T-lymphocyte differentiation, regulatory T cell development Sources: ISBN:0781735149 Relationships: is a type of T cell differentiation [GO:0030217] Subtypes: GO:0002307, GO:0002361